{
  "gene_symbol": "TRAF2",
  "term_id": "GO:0035591",
  "gene": "UniProtKB:Q12933",
  "gene_name": "TNF receptor-associated factor 2",
  "term_label": "signaling adaptor activity"
}